negative regulation of methanophenazine biosynthetic process [GO:1900963] (BP) Definition: Any process that stops, prevents or reduces the frequency, rate or extent of methanophenazine biosynthetic process. Relationships: is a type of negative regulation of biosynthetic process [GO:0009890]; is a type of regulation of methanophenazine biosynthetic process [GO:1900962]; negatively regulates methanophenazine biosynthetic process [GO:1900630] Also known as: down regulation of methanophenazine anabolism, down regulation of methanophenazine biosynthesis, down regulation of methanophenazine biosynthetic process, down regulation of methanophenazine formation, down regulation of methanophenazine synthesis, down-regulation of methanophenazine anabolism, down-regulation of methanophenazine biosynthesis, down-regulation of methanophenazine biosynthetic process, down-regulation of methanophenazine formation, down-regulation of methanophenazine synthesis, downregulation of methanophenazine anabolism, downregulation of methanophenazine biosynthesis, downregulation of methanophenazine biosynthetic process, downregulation of methanophenazine formation, downregulation of methanophenazine synthesis, inhibition of methanophenazine anabolism, inhibition of methanophenazine biosynthesis, inhibition of methanophenazine formation, inhibition of methanophenazine synthesis, negative regulation of methanophenazine anabolism, negative regulation of methanophenazine biosynthesis, negative regulation of methanophenazine formation, negative regulation of methanophenazine synthesis, inhibition of methanophenazine biosynthetic process Sources: GOC:TermGenie, GOC:mengo_curators